{
  "gene_symbol": "TMT1A",
  "gene_name": "N6-adenosine-methyltransferase TMT1A",
  "term_label": "methyltransferase activity",
  "term_id": "GO:0008168",
  "gene": "UniProtKB:Q9H8H3"
}